{
  "term_label": "I-SMAD binding",
  "term_id": "GO:0070411",
  "gene_name": "Mothers against decapentaplegic homolog 4",
  "gene": "UniProtKB:Q13485",
  "gene_symbol": "SMAD4"
}